{
  "gene_symbol": "HLTF",
  "term_label": "ATP-dependent activity, acting on DNA",
  "term_id": "GO:0008094",
  "gene_name": "Helicase-like transcription factor",
  "gene": "UniProtKB:Q14527"
}